galactitol 2-dehydrogenase activity [GO:0047713] (molecular function) Definition: Catalysis of the reaction: galactitol + NAD+ = D-tagatose + H+ + NADH. Sources: RHEA:20685 Relationships: is a type of oxidoreductase activity, acting on the CH-OH group of donors, NAD or NADP as acceptor [GO:0016616]; is a type of GO:0031320